{
  "gene_symbol": "APOBEC4",
  "term_id": "UNKNOWN:0002",
  "gene": "UniProtKB:Q8WW27",
  "gene_name": "Putative C-U-editing enzyme APOBEC-4",
  "term_label": "Unknown biological process"
}